{
  "gene_symbol": "URB1",
  "term_id": "GO:0000466",
  "gene_name": "Nucleolar pre-ribosomal-associated protein 1",
  "gene": "UniProtKB:O60287",
  "term_label": "maturation of 5.8S rRNA from tricistronic rRNA transcript (SSU-rRNA, 5.8S rRNA, LSU-rRNA)"
}